{
  "gene": "UniProtKB:Q99954",
  "term_id": "UNKNOWN:0003",
  "gene_symbol": "SMR3A",
  "term_label": "Unknown cellular component",
  "gene_name": "Submaxillary gland androgen-regulated protein 3A"
}